thermospermine catabolic process [GO:1903602] (biological process) Definition: The chemical reactions and pathways resulting in the breakdown of thermospermine. Also known as: thermospermine breakdown, thermospermine catabolism, thermospermine degradation Relationships: is a type of polyamine catabolic process [GO:0006598] References: PMID:24906355 Sources: GOC:TermGenie, GO_REF:0000068